{
  "term_label": "synapse",
  "gene": "UniProtKB:P0CG38",
  "gene_name": "POTE ankyrin domain family member I",
  "gene_symbol": "POTEI",
  "term_id": "GO:0045202"
}